brassinosteroid catabolic process [GO:0016133] (biological process) Relationships: is a type of GO:0016130; is a type of GO:0016131; is_a hormone catabolic process [GO:0042447] Definition: The chemical reactions and pathways resulting in the breakdown of brassinosteroids, any of a group of steroid derivatives that occur at very low concentrations in plant tissues and may have hormone-like effects. Sources: ISBN:0192801023 Also known as: brassinosteroid breakdown, brassinosteroid catabolism, brassinosteroid degradation